{
  "gene_name": "Phosphatidylinositol 3,4,5-trisphosphate 3-phosphatase and dual-specificity protein phosphatase PTEN",
  "term_label": "phosphatidylinositol-3,4,5-trisphosphate 3-phosphatase activity",
  "gene": "UniProtKB:P60484",
  "term_id": "GO:0016314",
  "gene_symbol": "PTEN"
}